{
  "term_label": "beta-catenin destruction complex",
  "term_id": "GO:0030877",
  "gene_symbol": "GSK3B",
  "gene_name": "Glycogen synthase kinase-3 beta",
  "gene": "UniProtKB:P49841"
}